{
  "gene_name": "Disco-interacting protein 2 homolog C",
  "gene_symbol": "DIP2C",
  "term_id": "UNKNOWN:0001",
  "gene": "UniProtKB:Q9Y2E4",
  "term_label": "Unknown molecular function"
}